{
  "gene": "UniProtKB:Q9C0A6",
  "term_label": "Unknown molecular function",
  "gene_symbol": "SETD5",
  "term_id": "UNKNOWN:0001",
  "gene_name": "Histone-lysine N-methyltransferase SETD5"
}